{
  "gene_symbol": "H2BC11",
  "gene_name": "Histone H2B type 1-J",
  "term_label": "antibacterial humoral response",
  "term_id": "GO:0019731",
  "gene": "UniProtKB:P06899"
}